guanyl deoxyribonucleotide binding [GO:0032560] (MF) Subtypes: dGMP binding [GO:0032565], dGDP binding [GO:0032566], dGTP binding [GO:0032567] Sources: GOC:mah Relationships: is a type of guanyl nucleotide binding [GO:0019001]; is a type of purine deoxyribonucleotide binding [GO:0032554] Definition: Binding to a guanyl deoxyribonucleotide, any compound consisting of guanosine esterified with (ortho)phosphate or an oligophosphate at any hydroxyl group on the deoxyribose moiety.